{
  "term_label": "cytoplasm",
  "gene_symbol": "PRKAB2",
  "gene": "UniProtKB:O43741",
  "gene_name": "5'-AMP-activated protein kinase subunit beta-2",
  "term_id": "GO:0005737"
}